synaptic vesicle transport along microtubule [GO:0099517] (biological process) Subtypes: anterograde synaptic vesicle transport [GO:0048490], retrograde synaptic vesicle transport [GO:0048491] Relationships: is a type of vesicle transport along microtubule [GO:0047496]; is a type of GO:0099514 Definition: The directed movement of synaptic vesicles along microtubules within a cell, powered by molecular motors. Sources: GOC:dos